specification of metanephric nephron tubule identity [GO:0072293] (biological process) Definition: The process in which the tubules arranged along the proximal/distal axis of the metanephric nephron acquire their identity. Sources: GOC:bf, GOC:mtg_kidney_jan10 Relationships: is a type of specification of nephron tubule identity [GO:0072081]; is a type of pattern specification involved in metanephros development [GO:0072268]; is part of proximal/distal pattern formation involved in metanephric nephron development [GO:0072272]; BFO_0000050 metanephric nephron tubule formation [GO:0072289] Subtypes: specification of metanephric connecting tubule identity [GO:0072294], GO:0072295, specification of metanephric loop of Henle identity [GO:0072296], specification of metanephric proximal tubule identity [GO:0072297]